{
  "term_label": "Unknown cellular component",
  "gene": "UniProtKB:O15466",
  "gene_name": "Alpha-2,8-sialyltransferase 8E",
  "gene_symbol": "ST8SIA5",
  "term_id": "UNKNOWN:0003"
}